new mitotic spindle pole body [GO:0071958] (CC) Relationships: is_a GO:0044732 References: PMID:15132994 Sources: GOC:mah, GOC:vw Also known as: new SPB Definition: The spindle pole body that is formed by spindle pole body duplication, and to which proteins involved in mitotic exit signaling (for example, the septation initiation network in fission yeast) localize.